adenine nucleotide transport [GO:0051503] (biological process) Relationships: is a type of GO:0015865 Subtypes: ADP transport [GO:0015866], GO:0015867, NAD transport [GO:0043132], GO:0046963, GO:0070730, GO:0071106, GO:0080121, GO:0140361, 5'-adenylyl sulfate transmembrane transport [GO:1902558] Definition: The directed movement of adenine nucleotides, ATP, ADP, and/or AMP, into, out of or within a cell, or between cells, by means of some agent such as a transporter or pore. Sources: GOC:ai